{
  "term_label": "Unknown molecular function",
  "gene_symbol": "UTP15",
  "term_id": "UNKNOWN:0001",
  "gene_name": "U3 small nucleolar RNA-associated protein 15 homolog",
  "gene": "UniProtKB:Q8TED0"
}